{
  "term_id": "GO:0007268",
  "gene_name": "Protein phosphatase 1 regulatory subunit 29",
  "term_label": "chemical synaptic transmission",
  "gene_symbol": "ELFN2",
  "gene": "UniProtKB:Q5R3F8"
}